right ventral flagellum [GO:0097559] (cellular component) Definition: A cilium (also called flagellum) found in Giardia species (trophozoite stage). It is nucleated by the right ventral basal body and exits the cell body proximally and dorsal to the ventral disc. Relationships: is_a GO:0097729 Also known as: right ventral cilium References: PMID:16607022, PMID:5961344 Sources: GOC:giardia, ISBN:9780124260207 Note: Note that we deem cilium and microtubule-based flagellum to be equivalent; the primary term name reflects frequency of use. Also note that, due to the asymmetric nature of the Giardia trophozoite, this term is defined spatially as the trophozoite is viewed from the dorsal side, with the two nuclei dorsal to the ventral disc, and the ventral disc toward the anterior.